{
  "gene": "UniProtKB:Q96HW7",
  "gene_name": "Integrator complex subunit 4",
  "gene_symbol": "INTS4",
  "term_id": "GO:0016180",
  "term_label": "snRNA processing"
}